{
  "term_id": "GO:0032922",
  "gene_name": "Circadian locomoter output cycles protein kaput",
  "term_label": "circadian regulation of gene expression",
  "gene": "UniProtKB:O15516",
  "gene_symbol": "CLOCK"
}